{
  "gene": "UniProtKB:Q8TDW0",
  "term_label": "volume-sensitive anion channel activity",
  "term_id": "GO:0005225",
  "gene_symbol": "LRRC8C",
  "gene_name": "Volume-regulated anion channel subunit LRRC8C"
}